{
  "gene_name": "Zinc finger and SCAN domain-containing protein 5A",
  "term_id": "GO:0000981",
  "gene_symbol": "ZSCAN5A",
  "gene": "UniProtKB:Q9BUG6",
  "term_label": "DNA-binding transcription factor activity, RNA polymerase II-specific"
}